{
  "term_id": "GO:0120200",
  "gene_name": "Retinal guanylyl cyclase 2",
  "term_label": "rod photoreceptor outer segment",
  "gene_symbol": "GUCY2F",
  "gene": "UniProtKB:P51841"
}